ER-dependent peroxisome localization [GO:0106101] (biological process) Definition: A process in which a protein is transported to, or maintained at, a location in a peroxisome via the endoplasmic reticulum. References: PMID:19479899, PMID:26408931 Sources: GOC:pga Relationships: is a type of protein localization to peroxisome [GO:0072662]